{
  "gene_symbol": "HYCC1",
  "term_label": "protein localization to plasma membrane",
  "gene": "UniProtKB:Q9BYI3",
  "gene_name": "Hyccin",
  "term_id": "GO:0072659"
}